{
  "term_label": "unfolded protein binding",
  "gene_name": "DnaJ homolog subfamily B member 2",
  "term_id": "GO:0051082",
  "gene": "UniProtKB:P25686",
  "gene_symbol": "DNAJB2"
}